{
  "term_label": "nucleosomal DNA binding",
  "term_id": "GO:0031492",
  "gene": "UniProtKB:Q5TEC6",
  "gene_name": "Histone H3-7",
  "gene_symbol": "H3-7"
}